{
  "term_id": "UNKNOWN:0002",
  "gene_symbol": "FAM30A",
  "gene_name": "Putative uncharacterized protein FAM30A",
  "term_label": "Unknown biological process",
  "gene": "UniProtKB:Q9NZY2"
}